{
  "gene_symbol": "MBD3L3",
  "term_label": "methyl-CpG binding",
  "term_id": "GO:0008327",
  "gene_name": "Putative methyl-CpG-binding domain protein 3-like 3",
  "gene": "UniProtKB:A6NE82"
}